negative regulation of B cell proliferation [GO:0030889] (biological process) Definition: Any process that stops, prevents or reduces the rate or extent of B cell proliferation. Sources: GOC:mah Also known as: down regulation of B cell proliferation, down-regulation of B cell proliferation, downregulation of B cell proliferation, negative regulation of B lymphocyte proliferation, negative regulation of B-cell proliferation, negative regulation of B-lymphocyte proliferation, inhibition of B cell proliferation Relationships: is a type of regulation of B cell proliferation [GO:0030888]; is_a negative regulation of lymphocyte proliferation [GO:0050672]; is a type of negative regulation of B cell activation [GO:0050869]; negatively regulates B cell proliferation [GO:0042100]